{
  "term_id": "GO:0005886",
  "gene": "UniProtKB:P48051",
  "gene_name": "G protein-activated inward rectifier potassium channel 2",
  "term_label": "plasma membrane",
  "gene_symbol": "KCNJ6"
}